centrosome [GO:0005813] (cellular component) Sources: GOC:mah, ISBN:0198547684 Relationships: is a type of microtubule organizing center [GO:0005815]; has part centriole [GO:0005814] Definition: A structure comprised of a core structure (in most organisms, a pair of centrioles) and peripheral material from which a microtubule-based structure, such as a spindle apparatus, is organized. Centrosomes occur close to the nucleus during interphase in many eukaryotic cells, though in animal cells it changes continually during the cell-division cycle. Subtypes: spindle pole centrosome [GO:0031616]